establishment of ommatidial planar polarity [GO:0042067] (biological process) Definition: The specification of polarized ommatidia. Ommatidia occur in two chiral forms. The trapezoidal arrangement of photoreceptors in the dorsal part of the eye is the mirror image of that in the ventral part. References: PMID:3076112, PMID:3937883 Sources: GOC:ascb_2009, GOC:dph, GOC:tb Relationships: is a type of GO:0001736; is a type of establishment or maintenance of cell polarity [GO:0007163]; is part of GO:0001745 Also known as: establishment of ommatidial polarity